{
  "gene_name": "Leukocyte immunoglobulin-like receptor subfamily B member 1",
  "term_id": "GO:0140105",
  "gene_symbol": "LILRB1",
  "gene": "UniProtKB:Q8NHL6",
  "term_label": "interleukin-10-mediated signaling pathway"
}